postganglionic parasympathetic fiber development [GO:0021784] (BP) Sources: GOC:cls, GOC:dgh, GOC:dph, GOC:jid, GO_REF:0000021 Relationships: is a type of GO:0048483; is part of GO:0007422; is part of parasympathetic nervous system development [GO:0048486] Definition: The process whose specific outcome is the progression of the postganglionic portion of the parasympathetic fiber over time, from its formation to the mature structure. The parasympathetic fiber is one of the two divisions of the vertebrate autonomic nervous system. Parasympathetic nerves emerge cranially as pre ganglionic fibers from oculomotor, facial, glossopharyngeal and vagus and from the sacral region of the spinal cord. Most neurons are cholinergic and responses are mediated by muscarinic receptors. The parasympathetic system innervates, for example: salivary glands, thoracic and abdominal viscera, bladder and genitalia.